{
  "gene_symbol": "BRIP1",
  "term_id": "GO:0003678",
  "gene_name": "Fanconi anemia group J protein",
  "term_label": "DNA helicase activity",
  "gene": "UniProtKB:Q9BX63"
}